{
  "gene": "UniProtKB:Q9H1J5",
  "gene_symbol": "WNT8A",
  "term_id": "GO:0005125",
  "gene_name": "Protein Wnt-8a",
  "term_label": "cytokine activity"
}